{
  "gene_name": "Speedy protein E6",
  "gene_symbol": "SPDYE6",
  "gene": "UniProtKB:P0CI01",
  "term_id": "GO:0019901",
  "term_label": "protein kinase binding"
}